{
  "term_label": "antigen binding",
  "term_id": "GO:0003823",
  "gene_name": "Immunoglobulin heavy variable 2-5",
  "gene_symbol": "IGHV2-5",
  "gene": "UniProtKB:P01817"
}